'de novo' GDP-L-fucose biosynthetic process [GO:0042351] (biological process) Definition: The chemical reactions and pathways resulting in the formation of GDP-L-fucose from GDP-D-mannose via GDP-4-dehydro-6-deoxy-D-mannose, requiring the functions of GDP-mannose 4,6-dehydratase (EC:4.2.1.47) and GDP-L-fucose synthase (EC:1.1.1.271). Relationships: is_a GO:0019673; is a type of GDP-L-fucose biosynthetic process [GO:0042350] Also known as: 'de novo' GDP-L-fucose anabolism, 'de novo' GDP-L-fucose biosynthesis, 'de novo' GDP-L-fucose formation, 'de novo' GDP-L-fucose synthesis, GDP-L-fucose biosynthesis, de novo pathway, GDP-L-fucose biosynthetic process, de novo pathway References: PMID:11030750